{
  "term_id": "UNKNOWN:0002",
  "gene": "UniProtKB:Q53FA7",
  "gene_name": "Quinone oxidoreductase PIG3",
  "gene_symbol": "TP53I3",
  "term_label": "Unknown biological process"
}